G protein-coupled adenosine receptor signaling pathway [GO:0001973] (biological process) Regulation: regulated by regulation of adenosine receptor signaling pathway [GO:0060167]; positively regulated by positive regulation of adenosine receptor signaling pathway [GO:0060168]; negatively regulated by negative regulation of adenosine receptor signaling pathway [GO:0060169] Sources: GOC:dph Relationships: is a type of G protein-coupled purinergic receptor signaling pathway [GO:0035588] Also known as: P1 receptor signaling pathway, adenosine receptor signaling pathway, G-protein coupled, adenosine receptor signalling pathway, adenosine receptor signaling pathway Definition: The series of molecular signals generated as a consequence of a receptor binding to extracellular adenosine and transmitting the signal to a heterotrimeric G-protein complex to initiate a change in cell activity.